{
  "gene_name": "Protein WFDC9",
  "term_label": "serine-type endopeptidase inhibitor activity",
  "gene": "UniProtKB:Q8NEX5",
  "term_id": "GO:0004867",
  "gene_symbol": "WFDC9"
}